{
  "term_label": "Unknown biological process",
  "term_id": "UNKNOWN:0002",
  "gene": "UniProtKB:Q4LEZ3",
  "gene_symbol": "AARD",
  "gene_name": "Alanine and arginine-rich domain-containing protein"
}